{
  "term_label": "cytoplasm",
  "gene_name": "Actin-related protein 5",
  "gene_symbol": "ACTR5",
  "term_id": "GO:0005737",
  "gene": "UniProtKB:Q9H9F9"
}